{
  "gene_symbol": "TRIM47",
  "gene_name": "E3 ubiquitin-protein ligase TRIM47",
  "gene": "UniProtKB:Q96LD4",
  "term_label": "Unknown cellular component",
  "term_id": "UNKNOWN:0003"
}